{
  "gene_name": "Olfactory receptor 2V2",
  "term_label": "olfactory receptor activity",
  "gene_symbol": "OR2V2",
  "gene": "UniProtKB:Q96R30",
  "term_id": "GO:0004984"
}